{
  "term_label": "nucleus",
  "gene": "UniProtKB:Q9H6B1",
  "gene_symbol": "ZNF385D",
  "gene_name": "Zinc finger protein 385D",
  "term_id": "GO:0005634"
}